detection of ethylene stimulus [GO:0009727] (BP) Definition: The series of events in which an ethylene (ethene) stimulus is received by a cell and converted into a molecular signal. Sources: GOC:sm Relationships: is a type of GO:0009720; is a type of response to ethylene [GO:0009723] Also known as: detection of ethene stimulus, perception of ethene stimulus, perception of ethylene stimulus